{
  "term_id": "GO:0016477",
  "gene_symbol": "SH3KBP1",
  "gene_name": "SH3 domain-containing kinase-binding protein 1",
  "gene": "UniProtKB:Q96B97",
  "term_label": "cell migration"
}